{
  "gene_symbol": "SFXN4",
  "gene_name": "Sideroflexin-4",
  "term_label": "mitochondrial inner membrane",
  "term_id": "GO:0005743",
  "gene": "UniProtKB:Q6P4A7"
}